{
  "gene": "UniProtKB:Q9NR63",
  "gene_name": "Cytochrome P450 26B1",
  "term_label": "central nervous system development",
  "term_id": "GO:0007417",
  "gene_symbol": "CYP26B1"
}